{
  "gene": "UniProtKB:O15164",
  "gene_symbol": "TRIM24",
  "gene_name": "Transcription intermediary factor 1-alpha",
  "term_label": "chromatin",
  "term_id": "GO:0000785"
}